siderophore uptake transmembrane transporter activity [GO:0015344] (molecular function) Definition: Enables the transfer of a solute or solutes from one side of a membrane to the other according to the reaction: siderophore-iron(ferrioxamine)(out) + H+(out) = siderophore-iron(ferrioxamine)(in) + H+(in). Sources: TC:2.A.1.16.1 Also known as: siderochrome-iron (ferrioxamine) uptake transporter, ferrioxamine uptake transmembrane transporter activity, siderophore-iron uptake transmembrane transporter activity Relationships: is_a siderophore-iron transmembrane transporter activity [GO:0015343]